{
  "term_label": "Unknown cellular component",
  "gene": "UniProtKB:Q13268",
  "term_id": "UNKNOWN:0003",
  "gene_symbol": "DHRS2",
  "gene_name": "Dehydrogenase_reductase SDR family member 2, mitochondrial"
}